{
  "term_label": "plasma membrane",
  "gene": "UniProtKB:Q9Y5G7",
  "gene_name": "Protocadherin gamma-A6",
  "term_id": "GO:0005886",
  "gene_symbol": "PCDHGA6"
}